{
  "term_label": "Unknown molecular function",
  "term_id": "UNKNOWN:0001",
  "gene_name": "Translin-associated factor X-interacting protein 1",
  "gene_symbol": "TSNAXIP1",
  "gene": "UniProtKB:Q2TAA8"
}